{
  "term_id": "GO:0007411",
  "gene_symbol": "EPHA3",
  "gene": "UniProtKB:P29320",
  "term_label": "axon guidance",
  "gene_name": "Ephrin type-A receptor 3"
}